{
  "gene": "UniProtKB:Q13571",
  "gene_symbol": "LAPTM5",
  "term_label": "lysosomal membrane",
  "gene_name": "Lysosomal-associated transmembrane protein 5",
  "term_id": "GO:0005765"
}